{
  "gene": "UniProtKB:Q03188",
  "gene_name": "Centromere protein C",
  "gene_symbol": "CENPC",
  "term_id": "UNKNOWN:0003",
  "term_label": "Unknown cellular component"
}